{
  "gene": "UniProtKB:P23490",
  "gene_name": "Loricrin",
  "gene_symbol": "LORICRIN",
  "term_label": "structural constituent of skin epidermis",
  "term_id": "GO:0030280"
}